{
  "gene_name": "Syntaxin-1A",
  "gene_symbol": "STX1A",
  "gene": "UniProtKB:Q16623",
  "term_id": "GO:0000149",
  "term_label": "SNARE binding"
}